meiotic metaphase I homologous chromosome alignment [GO:0043060] (biological process) Definition: A cell cycle process whereby homlogous chromosomes are positioned in a specific order and orientation at the metaphase plate (spindle equator) by the spindle machinery and centromere/kinetochore arrangement during meiosis I chromosome segregation. This alignment ensures that each daughter cell will receive the correct number of chromosomes during cell division. References: PMID:10809666 Also known as: meiotic metaphase I chromosome alignment Relationships: is a type of meiotic metaphase chromosome alignment [GO:0051311]; is part of homologous chromosome segregation [GO:0045143]